{
  "term_id": "GO:0020037",
  "gene_symbol": "HBE1",
  "gene_name": "Hemoglobin subunit epsilon",
  "term_label": "heme binding",
  "gene": "UniProtKB:P02100"
}